{
  "gene": "UniProtKB:P23975",
  "term_id": "GO:0042734",
  "gene_name": "Sodium-dependent noradrenaline transporter",
  "gene_symbol": "SLC6A2",
  "term_label": "presynaptic membrane"
}